late endosome to vacuole transport via multivesicular body sorting pathway [GO:0032511] (biological process) Definition: The directed movement of substances from endosomes to vacuoles by a pathway in which molecules are sorted into multivesicular bodies, which then fuse with the vacuole. Subtypes: protein transport to vacuole involved in ubiquitin-dependent protein catabolic process via the multivesicular body sorting pathway [GO:0043328] References: PMID:12461556, PMID:16689637 Sources: GOC:mah Also known as: endosome to vacuole transport via MVB sorting pathway Relationships: is a type of endosome transport via multivesicular body sorting pathway [GO:0032509]; is a type of late endosome to vacuole transport [GO:0045324]